{
  "term_id": "UNKNOWN:0001",
  "gene_symbol": "RTL9",
  "gene_name": "Retrotransposon Gag-like protein 9",
  "term_label": "Unknown molecular function",
  "gene": "UniProtKB:Q8NET4"
}